{
  "gene_name": "Guanine nucleotide-binding protein G(q) subunit alpha",
  "gene": "UniProtKB:P50148",
  "gene_symbol": "GNAQ",
  "term_label": "adenylate cyclase-activating G protein-coupled receptor signaling pathway",
  "term_id": "GO:0007189"
}